{
  "gene": "UniProtKB:P46098",
  "term_label": "regulation of membrane potential",
  "gene_name": "5-hydroxytryptamine receptor 3A",
  "term_id": "GO:0042391",
  "gene_symbol": "HTR3A"
}